{
  "gene": "UniProtKB:Q04759",
  "gene_symbol": "PRKCQ",
  "term_id": "GO:0004674",
  "gene_name": "Protein kinase C theta type",
  "term_label": "protein serine/threonine kinase activity"
}